{
  "gene_name": "Protein transport protein Sec24C",
  "gene": "UniProtKB:P53992",
  "gene_symbol": "SEC24C",
  "term_id": "GO:0000149",
  "term_label": "SNARE binding"
}